insulin binding [GO:0043559] (molecular function) Definition: Binding to insulin, a polypeptide hormone produced by the islets of Langerhans of the pancreas in mammals, and by the homologous organs of other organisms. Sources: ISBN:0198506732 Relationships: is_a protein binding [GO:0005515]; is_a peptide hormone binding [GO:0017046]